double-strand break repair via synthesis-dependent strand annealing [GO:0045003] (biological process) Definition: SDSA is a major mechanism of double-strand break repair in mitosis which allows for the error-free repair of a double-strand break without the exchange of adjacent sequences. The broken DNA searches for and base pairs with a homologous region in an intact chromosome. DNA synthesis initiates from the 3' end of the invading DNA strand, using the intact chromosome as the template. Newly synthesized DNA is then displaced from the template and anneal with its complement on the other side of the double-strand break. Relationships: is a type of double-strand break repair via homologous recombination [GO:0000724] References: PMID:10357855 Also known as: SDSA, mitotic gene conversion